{
  "term_label": "zinc ion binding",
  "gene_name": "LITAF domain-containing protein",
  "gene": "UniProtKB:A0A1B0GVX0",
  "gene_symbol": "LITAFD",
  "term_id": "GO:0008270"
}